{
  "term_id": "GO:0005200",
  "gene_name": "Lamin-B1",
  "gene_symbol": "LMNB1",
  "gene": "UniProtKB:P20700",
  "term_label": "structural constituent of cytoskeleton"
}